alpha-N-acetylgalactosaminidase activity [GO:0008456] (molecular function) Also known as: N-acetyl-alpha-D-galactosaminidase activity, N-acetyl-alpha-galactosaminidase activity, alpha-N-acetyl-D-galactosaminide N-acetylgalactosaminohydrolase activity, alpha-NAGA activity, alpha-acetylgalactosaminidase activity, alpha-galactosidase B activity Relationships: is a type of hexosaminidase activity [GO:0015929] Sources: EC:3.2.1.49 Definition: Catalysis of the hydrolysis of terminal non-reducing N-acetyl-D-galactosamine residues in N-acetyl-alpha-D-galactosaminides.